{
  "term_label": "spermatid development",
  "gene": "UniProtKB:P04554",
  "gene_symbol": "PRM2",
  "term_id": "GO:0007286",
  "gene_name": "Protamine-2"
}